{
  "gene_symbol": "SLC16A7",
  "gene": "UniProtKB:O60669",
  "gene_name": "Monocarboxylate transporter 2",
  "term_id": "GO:0015129",
  "term_label": "lactate transmembrane transporter activity"
}